{
  "gene_symbol": "SEC16A",
  "term_label": "endoplasmic reticulum exit site",
  "gene": "UniProtKB:O15027",
  "term_id": "GO:0070971",
  "gene_name": "Protein transport protein Sec16A"
}